{
  "term_id": "GO:0034551",
  "gene_symbol": "TTC19",
  "term_label": "mitochondrial respiratory chain complex III assembly",
  "gene": "UniProtKB:Q6DKK2",
  "gene_name": "Tetratricopeptide repeat protein 19, mitochondrial"
}